{
  "gene": "UniProtKB:Q6ZRG5",
  "gene_name": "Putative uncharacterized protein FLJ43944",
  "term_label": "Unknown biological process",
  "term_id": "UNKNOWN:0002",
  "gene_symbol": "Q6ZRG5"
}